{
  "gene_name": "Endoplasmic reticulum-Golgi intermediate compartment protein 3",
  "term_id": "GO:0006890",
  "gene": "UniProtKB:Q9Y282",
  "gene_symbol": "ERGIC3",
  "term_label": "retrograde vesicle-mediated transport, Golgi to endoplasmic reticulum"
}